copal-8-ol diphosphate(3-) biosynthetic process [GO:1902243] (biological process) Also known as: copal-8-ol diphosphate(3-) anabolism, copal-8-ol diphosphate(3-) biosynthesis, copal-8-ol diphosphate(3-) formation, copal-8-ol diphosphate(3-) synthesis References: PMID:22672125 Sources: GOC:TermGenie Relationships: is a type of phospholipid biosynthetic process [GO:0008654]; is a type of diterpenoid biosynthetic process [GO:0016102] Definition: The chemical reactions and pathways resulting in the formation of copal-8-ol diphosphate(3-).